positive regulation of neutrophil mediated killing of symbiont cell [GO:0070961] (biological process) Subtypes: positive regulation of neutrophil mediated killing of bacterium [GO:0070962], GO:0070965 Sources: GOC:add, GOC:mah Relationships: is a type of positive regulation of response to biotic stimulus [GO:0002833]; is_a GO:0031349; is a type of positive regulation of response to external stimulus [GO:0032103]; is a type of positive regulation of killing of cells of another organism [GO:0051712]; is a type of regulation of neutrophil mediated killing of symbiont cell [GO:0070949]; is_a positive regulation of neutrophil mediated cytotoxicity [GO:0070960]; positively regulates neutrophil-mediated killing of symbiont cell [GO:0070943] Also known as: up regulation of neutrophil mediated killing of symbiont cell, up-regulation of neutrophil mediated killing of symbiont cell, upregulation of neutrophil mediated killing of symbiont cell, activation of neutrophil mediated killing of symbiont cell, stimulation of neutrophil mediated killing of symbiont cell Definition: Any process that increases the frequency, rate or extent of the directed killing of a symbiont target cell by a neutrophil.